1-methyladenosine nucleosidase activity [GO:0047518] (MF) Relationships: is a type of hydrolase activity, hydrolyzing N-glycosyl compounds [GO:0016799] Definition: Catalysis of the reaction: 1-methyladenosine + H2O = 1-methyladenine + ribofuranose. Sources: EC:3.2.2.13, RHEA:12865 Also known as: 1-methyladenosine hydrolase activity, 1-methyladenosine ribohydrolase activity